metanephros morphogenesis [GO:0003338] (biological process) Definition: The process in which the anatomical structures of the metanephros are generated and organized. Sources: GOC:dph, GOC:yaf Relationships: is a type of GO:0060993; is part of GO:0001656